surface coat of collagen and cuticulin-based cuticle extracellular matrix [GO:0060104] (cellular component) Definition: An electron dense, amorphous envelope that comprises the outermost layer of the cuticle. The surface coat is loosely apposed to the epicuticle, has distinct biochemical properties, is synthesized by cells other than the underlying hypodermis, and is labile. In addition to serving as a lubricant to protect against abrasion and dehydration, the surface coat may also play important roles in infection and immune evasion. An example of this component is found in Caenorhabditis elegans. Also known as: surface coat of collagen and cuticulin-based exoskeleton extracellular matrix Relationships: is a type of cellular anatomical structure [GO:0110165]; is part of GO:0060102 Sources: GOC:dph, GOC:kmv, ISSN:15518507